4-hydroxy-3-methylbut-2-enyl-diphosphate synthase activity (flavodoxin) [GO:0141197] (molecular function) Also known as: (E)-4-hydroxy-3-methylbut-2-enyl diphosphate synthase activity, 4-hydroxy-3-methylbut-2-en-1-yl diphosphate synthase activity Definition: Catalysis of the reaction: (2E)-4-hydroxy-3-methylbut-2-enyl diphosphate + 2 H+ + H2O + oxidized [flavodoxin] = 2-C-methyl-D-erythritol 2,4-cyclic diphosphate + reduced [flavodoxin]. Relationships: is a type of oxidoreductase activity, acting on CH or CH2 groups, with an iron-sulfur protein as acceptor [GO:0052592] Sources: RHEA:43604